{
  "term_id": "GO:0002486",
  "gene_name": "Zinc-alpha-2-glycoprotein",
  "gene": "UniProtKB:P25311",
  "gene_symbol": "AZGP1",
  "term_label": "antigen processing and presentation of endogenous peptide antigen via MHC class I via ER pathway, TAP-independent"
}